NAD(P)HX epimerase activity [GO:0052856] (molecular function) Definition: Catalysis of the reactions: (6R)-NADHX = (6S)-NADHX and (6R)-NADPHX = (6S)-NADPHX. References: PMID:21994945 Sources: EC:5.1.99.6 Also known as: NADHX epimerase activity, NADPHX epimerase activity Relationships: is a type of racemase and epimerase activity [GO:0016854]